trimetaphosphatase activity [GO:0050351] (molecular function) Relationships: is a type of GO:0016818 Also known as: inorganic trimetaphosphatase activity, trimetaphosphate hydrolase activity Sources: EC:3.6.1.2, RHEA:11088 Definition: Catalysis of the reaction: H2O + trimetaphosphate = 2 H+ + triphosphate.